NOXA-BCL-2 complex [GO:0097147] (cellular component) Relationships: is a type of GO:0097136 Definition: A heterodimeric protein complex consisting of NOXA and BCL-2, members of the Bcl-2 family of anti- and proapoptotic regulators. References: PMID:14634621 Sources: GOC:so